{
  "term_label": "NLS-bearing protein import into nucleus",
  "term_id": "GO:0006607",
  "gene_name": "RANBP2-like and GRIP domain-containing protein 5_6",
  "gene_symbol": "RGPD5",
  "gene": "UniProtKB:Q99666"
}